regulation of hepatocyte apoptotic process [GO:1903943] (BP) Also known as: regulation of hepatocyte apoptosis Subtypes: negative regulation of hepatocyte apoptotic process [GO:1903944], positive regulation of hepatocyte apoptotic process [GO:1903945] Definition: Any process that modulates the frequency, rate or extent of hepatocyte apoptotic process. Relationships: is a type of regulation of epithelial cell apoptotic process [GO:1904035]; regulates hepatocyte apoptotic process [GO:0097284] References: PMID:8649852 Sources: GOC:TermGenie, GO_REF:0000058